{
  "term_id": "GO:0000978",
  "gene_name": "Zinc finger protein 565",
  "gene": "UniProtKB:Q8N9K5",
  "term_label": "RNA polymerase II cis-regulatory region sequence-specific DNA binding",
  "gene_symbol": "ZNF565"
}